{
  "term_id": "GO:0002181",
  "term_label": "cytoplasmic translation",
  "gene_symbol": "RPL9P9",
  "gene": "UniProtKB:P32969",
  "gene_name": "Large ribosomal subunit protein uL6"
}